{
  "term_id": "GO:0005922",
  "gene": "UniProtKB:Q8NFK1",
  "gene_symbol": "GJC3",
  "term_label": "connexin complex",
  "gene_name": "Gap junction gamma-3 protein"
}